{
  "gene": "UniProtKB:Q0VF49",
  "gene_symbol": "KIAA2012",
  "term_label": "Unknown biological process",
  "term_id": "UNKNOWN:0002",
  "gene_name": "Uncharacterized protein KIAA2012"
}